{
  "gene_symbol": "H2BC5",
  "gene_name": "Histone H2B type 1-D",
  "term_label": "extracellular space",
  "gene": "UniProtKB:P58876",
  "term_id": "GO:0005615"
}